halimadienyl-diphosphate synthase activity [GO:0035439] (molecular function) Definition: Catalysis of the reaction: geranylgeranyl diphosphate = halima-5(6),13-dien-15-yl diphosphate. Also known as: halima-5(6),13-dien-15-yl-diphosphate lyase (cyclizing), halimadienyl diphosphate synthase activity Sources: EC:5.5.1.16 Relationships: is a type of cyclase activity [GO:0009975]; is a type of GO:0016872